{
  "gene_symbol": "PCYT1B",
  "term_label": "choline-phosphate cytidylyltransferase activity",
  "term_id": "GO:0004105",
  "gene_name": "Choline-phosphate cytidylyltransferase B",
  "gene": "UniProtKB:Q9Y5K3"
}